{
  "gene_name": "Glutamate receptor ionotropic, kainate 4",
  "gene": "UniProtKB:Q16099",
  "term_id": "GO:1904315",
  "gene_symbol": "GRIK4",
  "term_label": "transmitter-gated monoatomic ion channel activity involved in regulation of postsynaptic membrane potential"
}